cornea development in camera-type eye [GO:0061303] (biological process) Sources: GOC:dph Relationships: is a type of anatomical structure development [GO:0048856]; is part of camera-type eye development [GO:0043010] Subtypes: avascular cornea development in camera-type eye [GO:0036331] Definition: The progression of the cornea over time, from its formation to the mature structure. The cornea is the transparent structure that covers the anterior of the eye.